dendritic branch point [GO:1990033] (cellular component) Relationships: is a type of neuron projection branch point [GO:0061845]; BFO_0000050 dendritic tree [GO:0097447] Also known as: branch point of dendrite Sources: GOC:aruk, GOC:bc, NIF_Subcellular:sao1348591767 Definition: The part of a dendritic tree where it branches, giving rise to a dendritic branch.